response to acid chemical [GO:0001101] (biological process) Definition: Any process that results in a change in state or activity of a cell or an organism (in terms of movement, secretion, enzyme production, gene expression, etc.) as a result of a stimulus by the chemical structure of the anion portion of a dissociated acid (rather than the acid acting as a proton donor). The acid chemical may be in gaseous, liquid or solid form. Sources: GOC:go_curators, GOC:rn Also known as: response to acid, response to acid anion, response to oxoanion Note: This term should be used to describe a response to a specific acid as a chemical. E.g., if an organism were responding to glutamate, then the response would be glutamate-specific; the organism is actually responding to the chemical structure of the anion portion of the dissociated acid. Note that this term is in the subset of terms that should not be used for direct gene product annotation. Instead, select a child term or, if no appropriate child term exists, please request a new term. Direct annotations to this term may be amended during annotation QC. If annotating experiments where an acid is playing a role as a proton donor, please annotate to GO:0010447 'response to acidic pH' instead. Relationships: is a type of GO:0042221 Subtypes: GO:0009415, response to amino acid [GO:0043200], cellular response to acid chemical [GO:0071229], stress response to acid chemical [GO:0097532]